{
  "gene": "UniProtKB:P48436",
  "gene_name": "Transcription factor SOX-9",
  "gene_symbol": "SOX9",
  "term_label": "morphogenesis of an epithelium",
  "term_id": "GO:0002009"
}